histone H1K26me2 reader activity [GO:0160268] (molecular function) Relationships: is_a histone H1 reader activity [GO:0140128] References: PMID:17540172 Definition: A histone reader that recognizes a histone H1 dimethylated at lysine 26.